single-strand break repair via homologous recombination [GO:1990396] (biological process) Definition: The error-free repair of a single-strand break in DNA in which the broken DNA molecule is repaired using homologous sequences. A strand in the broken DNA searches for a homologous region in an intact chromosome to serve as the template for DNA synthesis. The restoration of two intact DNA molecules results in the exchange, reciprocal or nonreciprocal, of genetic material between the intact DNA molecule and the broken DNA molecule. References: PMID:24339919 Sources: GOC:bhm Relationships: is a type of GO:0000012; is a type of GO:0000725; is a type of error-free postreplication DNA repair [GO:0042275] Regulation: regulated by regulation of single-strand break repair via homologous recombination [GO:1903110]; negatively regulated by negative regulation of single-strand break repair via homologous recombination [GO:1903111]; positively regulated by GO:1903112